serotonin binding [GO:0051378] (molecular function) Definition: Binding to serotonin (5-hydroxytryptamine), a monoamine neurotransmitter occurring in the peripheral and central nervous systems, also having hormonal properties. Sources: GOC:ai Relationships: is a type of cation binding [GO:0043169]; is a type of amine binding [GO:0043176]; is a type of GO:1901363 Also known as: 5-hydroxytryptamine binding